{
  "gene": "UniProtKB:Q9ULM6",
  "gene_name": "CCR4-NOT transcription complex subunit 6",
  "gene_symbol": "CNOT6",
  "term_id": "UNKNOWN:0003",
  "term_label": "Unknown cellular component"
}